cellular response to quercetin [GO:1905236] (biological process) References: PMID:24914722 Sources: GOC:TermGenie, GO_REF:0000071 Relationships: is a type of response to quercetin [GO:1905235]; is a type of cellular response to flavonoid [GO:1905396] Definition: Any process that results in a change in state or activity of a cell (in terms of movement, secretion, enzyme production, gene expression, etc.) as a result of a quercetin stimulus.